negative regulation of response to drug [GO:2001024] (BP) Relationships: is a type of GO:0048585; is_a regulation of response to drug [GO:2001023]; negatively regulates response to xenobiotic stimulus [GO:0009410] Also known as: negative regulation of drug resistance, negative regulation of drug susceptibility/resistance Subtypes: negative regulation of xenobiotic detoxification by transmembrane export across the plasma membrane [GO:1905700], negative regulation of cellular response to drug [GO:2001039] Definition: Any process that stops, prevents or reduces the frequency, rate or extent of response to drug. Sources: GOC:obol